negative regulation of exit from mitosis [GO:0001100] (biological process) Relationships: is a type of GO:0007096; is a type of negative regulation of mitotic cell cycle phase transition [GO:1901991]; negatively regulates exit from mitosis [GO:0010458] Subtypes: mitotic spindle orientation checkpoint signaling [GO:0031578] Also known as: down regulation of exit from mitosis, down-regulation of exit from mitosis, downregulation of exit from mitosis, inhibition of exit from mitosis Sources: GOC:rn Definition: Any process involved in the inhibition of progression from anaphase/telophase (high mitotic CDK activity) to G1 (low mitotic CDK activity).